{
  "gene_symbol": "ST8SIA4",
  "gene_name": "CMP-N-acetylneuraminate-poly-alpha-2,8-sialyltransferase",
  "term_label": "Unknown cellular component",
  "term_id": "UNKNOWN:0003",
  "gene": "UniProtKB:Q92187"
}